{
  "gene": "UniProtKB:P28356",
  "term_label": "regulation of transcription by RNA polymerase II",
  "gene_name": "Homeobox protein Hox-D9",
  "term_id": "GO:0006357",
  "gene_symbol": "HOXD9"
}